{
  "gene": "UniProtKB:Q9H1V8",
  "term_id": "GO:0015820",
  "gene_symbol": "SLC6A17",
  "term_label": "L-leucine transport",
  "gene_name": "Sodium-dependent neutral amino acid transporter SLC6A17"
}